{
  "gene_name": "ADP-ribosylation factor-like protein 8A",
  "term_id": "UNKNOWN:0001",
  "gene_symbol": "ARL8A",
  "term_label": "Unknown molecular function",
  "gene": "UniProtKB:Q96BM9"
}